K11-linked polyubiquitin modification-dependent protein binding [GO:0071795] (MF) Relationships: is a type of polyubiquitin modification-dependent protein binding [GO:0031593] References: PMID:18775313 Sources: GOC:sp Definition: Binding to a protein upon poly-ubiquitination formed by linkages between lysine residues at position 11 in the target protein.